{
  "gene": "UniProtKB:P14616",
  "term_label": "insulin receptor activity",
  "term_id": "GO:0005009",
  "gene_name": "Insulin receptor-related protein",
  "gene_symbol": "INSRR"
}